proximal neuron projection [GO:1990769] (CC) Definition: The portion of an axon or dendrite that is close to the neuronal cell body. References: PMID:21104189 Relationships: is a type of neuron projection [GO:0043005]